{
  "term_id": "GO:0016064",
  "term_label": "immunoglobulin mediated immune response",
  "gene": "UniProtKB:A0A087WSY4",
  "gene_symbol": "IGHV4-30-2",
  "gene_name": "Immunoglobulin heavy variable 4-30-2"
}